{
  "gene": "UniProtKB:Q9BQG2",
  "gene_name": "NAD-capped RNA hydrolase NUDT12",
  "gene_symbol": "NUDT12",
  "term_label": "peroxisome",
  "term_id": "GO:0005777"
}